{
  "term_label": "cytosol",
  "term_id": "GO:0005829",
  "gene": "UniProtKB:P35813",
  "gene_name": "Protein phosphatase 1A",
  "gene_symbol": "PPM1A"
}